{
  "gene_name": "Peroxisome assembly protein 12",
  "gene_symbol": "PEX12",
  "term_id": "GO:1990429",
  "term_label": "peroxisomal importomer complex",
  "gene": "UniProtKB:O00623"
}